{
  "gene": "UniProtKB:Q9Y561",
  "gene_name": "Low-density lipoprotein receptor-related protein 12",
  "gene_symbol": "LRP12",
  "term_id": "GO:0005886",
  "term_label": "plasma membrane"
}